{
  "gene_symbol": "ZNF239",
  "gene_name": "Zinc finger protein 239",
  "term_id": "GO:0000981",
  "gene": "UniProtKB:Q16600",
  "term_label": "DNA-binding transcription factor activity, RNA polymerase II-specific"
}